{
  "term_id": "GO:0000978",
  "term_label": "RNA polymerase II cis-regulatory region sequence-specific DNA binding",
  "gene_name": "Zinc finger protein 264",
  "gene_symbol": "ZNF264",
  "gene": "UniProtKB:O43296"
}